axonemal microtubule depolymerization [GO:0060404] (biological process) Definition: The removal of tubulin heterodimers from one or both ends of an axonemal microtubule. An axonemal microtubule is a microtubule in the axoneme of a cilium or flagellum; an axoneme contains nine modified doublet microtubules surrounding a pair of single microtubules. Sources: GOC:cilia, GOC:dph, GOC:krc, GOC:tb Relationships: is a type of cytoplasmic microtubule depolymerization [GO:0010938]; is a type of cilium disassembly [GO:0061523]; occurs in axoneme [GO:0005930] Regulation: negatively regulated by GO:0007027